hypothalamus development [GO:0021854] (biological process) Definition: The progression of the hypothalamus region of the forebrain, from its initial formation to its mature state. Sources: GOC:cls, GOC:dgh, GOC:dph, GOC:jid, GO_REF:0000021 Relationships: is a type of GO:0048856; is part of GO:0021536; is part of limbic system development [GO:0021761]